{
  "term_id": "UNKNOWN:0003",
  "term_label": "Unknown cellular component",
  "gene_symbol": "TMEM74B",
  "gene": "UniProtKB:Q9NUR3",
  "gene_name": "Transmembrane protein 74B"
}